serotonergic synapse [GO:0099154] (cellular component) Definition: A synapse that uses serotonin as a neurotransmitter. Relationships: is a type of synapse [GO:0045202] Sources: GOC:dos